{
  "gene_name": "G-protein coupled receptor family C group 5 member D",
  "gene_symbol": "GPRC5D",
  "term_id": "GO:0030295",
  "gene": "UniProtKB:Q9NZD1",
  "term_label": "protein kinase activator activity"
}